{
  "gene_symbol": "FBXW2",
  "term_id": "UNKNOWN:0001",
  "term_label": "Unknown molecular function",
  "gene": "UniProtKB:Q9UKT8",
  "gene_name": "F-box_WD repeat-containing protein 2"
}